response to melanocyte-stimulating hormone [GO:1990680] (biological process) Also known as: response to MSH Relationships: is a type of response to peptide hormone [GO:0043434] Definition: Any process that results in a change in state or activity of a cell or an organism (in terms of movement, secretion, enzyme production, gene expression, etc.) as a result of a melanocyte-stimulating hormone stimulus. The binding of any one of three melanocyte-stimulating hormones causes dispersal of melanosomes in melanophores of poikilothermic vertebrates. References: PMID:17036007